positive regulation of cordyol C biosynthetic process [GO:1900863] (biological process) Relationships: is a type of positive regulation of secondary metabolite biosynthetic process [GO:1900378]; is a type of regulation of cordyol C biosynthetic process [GO:1900861]; positively regulates cordyol C biosynthetic process [GO:1900799] Definition: Any process that activates or increases the frequency, rate or extent of cordyol C biosynthetic process. Also known as: up regulation of cordyol C biosynthetic process, up-regulation of cordyol C biosynthetic process, upregulation of cordyol C biosynthetic process, activation of cordyol C biosynthetic process Sources: GOC:TermGenie, GOC:di